{
  "term_id": "GO:0051117",
  "gene_name": "V-type proton ATPase 116 kDa subunit a 4",
  "gene_symbol": "ATP6V0A4",
  "term_label": "ATPase binding",
  "gene": "UniProtKB:Q9HBG4"
}